baroreceptor detection of increased arterial stretch [GO:0003023] (biological process) Sources: GOC:mtg_cardio Definition: The series of events by which an increase in diameter of an artery is detected and converted to a molecular signal. Relationships: is a type of baroreceptor detection of arterial stretch [GO:0001981]; BFO_0000050 baroreceptor response to increased systemic arterial blood pressure [GO:0001983]